maturation of 5.8S rRNA from tetracistronic rRNA transcript (SSU-rRNA, 5.8S rRNA, 2S rRNA, LSU-rRNA) [GO:0000487] (biological process) Sources: GOC:curators Relationships: is a type of GO:0000460 Definition: Any process involved in the maturation of a precursor 5.8S ribosomal RNA (rRNA) molecule into a mature 5.8S rRNA molecule from the pre-rRNA molecule originally produced as a tetracistronic rRNA transcript that contains the Small Subunit (SSU) rRNA, the 8.8S rRNA, the 2S rRNA, and the Large Subunit (LSU) in that order from 5' to 3' along the primary transcript.